{
  "term_id": "GO:0005886",
  "gene": "UniProtKB:Q8TDU6",
  "gene_symbol": "GPBAR1",
  "gene_name": "G-protein coupled bile acid receptor 1",
  "term_label": "plasma membrane"
}